{
  "term_id": "UNKNOWN:0001",
  "term_label": "Unknown molecular function",
  "gene_name": "Proline-rich protein 23E",
  "gene_symbol": "PRR23E",
  "gene": "UniProtKB:Q8N813"
}